{
  "term_id": "GO:0008284",
  "gene_name": "Interleukin-11",
  "term_label": "positive regulation of cell population proliferation",
  "gene_symbol": "IL11",
  "gene": "UniProtKB:P20809"
}